{
  "gene_symbol": "TRAFD1",
  "term_id": "GO:0005739",
  "gene": "UniProtKB:O14545",
  "gene_name": "TRAF-type zinc finger domain-containing protein 1",
  "term_label": "mitochondrion"
}